biological process involved in symbiotic interaction [GO:0044403] (biological process) Regulation: regulated by GO:0043903 Also known as: commensalism, host-pathogen interaction, parasitism, symbiosis, symbiosis, encompassing mutualism through parasitism, symbiotic interaction, symbiotic interaction between host and organism, symbiotic interaction between organisms, symbiotic interaction between species, symbiotic process Subtypes: GO:0036377, multi-species biofilm formation [GO:0044399], biological process involved in interaction with host [GO:0051701], GO:0051702, intracellular transport of virus [GO:0075733], GO:0085030 Relationships: is a type of biological process involved in interspecies interaction between organisms [GO:0044419] References: PMID:31257129 Sources: GOC:cc Definition: A process carried out by gene products in an organism that enable the organism to engage in a symbiotic relationship, a more or less intimate association, with another organism. The various forms of symbiosis include parasitism, in which the association is disadvantageous or destructive to one of the organisms; mutualism, in which the association is advantageous, or often necessary to one or both and not harmful to either; and commensalism, in which one member of the association benefits while the other is not affected. However, mutualism, parasitism, and commensalism are often not discrete categories of interactions and should rather be perceived as a continuum of interaction ranging from parasitism to mutualism. In fact, the direction of a symbiotic interaction can change during the lifetime of the symbionts due to developmental changes as well as changes in the biotic/abiotic environment in which the interaction occurs. Microscopic symbionts are often referred to as endosymbionts.